regulation of cell differentiation involved in embryonic placenta development [GO:0060800] (biological process) Relationships: is a type of GO:0045595; is a type of regulation of reproductive process [GO:2000241]; regulates cell differentiation involved in embryonic placenta development [GO:0060706] Definition: Any process that modulates the rate, frequency or extent of cell differentiation that contributes to the progression of the placenta over time, from its initial condition to its mature state. Sources: GOC:dph, GOC:sdb_2009, GOC:tb Subtypes: negative regulation of cell differentiation involved in embryonic placenta development [GO:0060806]